protein localization to meiotic spindle [GO:1905359] (biological process) Relationships: is a type of protein localization to microtubule cytoskeleton [GO:0072698] References: PMID:26696398 Sources: GOC:TermGenie, GO_REF:0000087 Definition: A process in which a protein is transported to, or maintained in, a location within a meiotic spindle. Subtypes: protein localization to meiotic spindle midzone [GO:1903096] Also known as: protein localisation to meiotic spindle